{
  "gene_name": "Cytochrome b-c1 complex subunit 10",
  "gene_symbol": "UQCR11",
  "gene": "UniProtKB:O14957",
  "term_label": "Unknown biological process",
  "term_id": "UNKNOWN:0002"
}